acyl-CoA metabolic process [GO:0006637] (biological process) Also known as: acyl-CoA metabolism Subtypes: acetyl-CoA metabolic process [GO:0006084], succinyl-CoA metabolic process [GO:0006104], fatty-acyl-CoA metabolic process [GO:0035337], L-methylmalonyl-CoA metabolic process [GO:0046491], acyl-CoA biosynthetic process [GO:0071616], benzoyl-CoA metabolic process [GO:1901787], 2-hydroxybenzoyl-CoA catabolic process [GO:1901886], malonyl-CoA metabolic process [GO:2001293] Sources: ISBN:0198506732 Definition: The chemical reactions and pathways involving acyl-CoA, any derivative of coenzyme A in which the sulfhydryl group is in thiolester linkage with an acyl group. Relationships: is a type of nucleoside phosphate metabolic process [GO:0006753]; is a type of sulfur compound metabolic process [GO:0006790]; is a type of amide metabolic process [GO:0043603]; is a type of purine-containing compound metabolic process [GO:0072521]